{
  "term_id": "GO:0030425",
  "gene": "UniProtKB:Q09470",
  "gene_name": "Potassium voltage-gated channel subfamily A member 1",
  "gene_symbol": "KCNA1",
  "term_label": "dendrite"
}